organohalogen metabolic process [GO:0090345] (biological process) Definition: The chemical reactions and pathways involving organohalogen compounds, as carried out by individual cells. Regulation: regulated by regulation of organohalogen metabolic process [GO:0090347] Relationships: is a type of GO:0008152 Sources: GOC:BHF Subtypes: bromoxynil metabolic process [GO:0018881], GO:0018888, 2,4-dichlorophenoxyacetic acid metabolic process [GO:0018901], GO:0018911, chlorobenzene catabolic process [GO:0018914], iprodione metabolic process [GO:0018922], 1,4-dichlorobenzene catabolic process [GO:0019261], pentachlorophenol catabolic process [GO:0019338], atrazine catabolic process [GO:0019381], 1-(3,5-dichloro-2,6-dihydroxy-4-methoxyphenyl)hexan-1-one metabolic process [GO:0031147], halogenated hydrocarbon metabolic process [GO:0042197], 2,4,5-trichlorophenoxyacetic acid catabolic process [GO:0046228], 2,4-dichlorobenzoate catabolic process [GO:0046298], 2-chloro-N-isopropylacetanilide catabolic process [GO:0046302], GO:0090346, GO:0140878, ochratoxin A catabolic process [GO:1900817], ochratoxin A biosynthetic process [GO:1900818], 3-chlorocatechol catabolic process [GO:1901168], 3-chlorocatechol biosynthetic process [GO:1901169]